mesenchymal cell differentiation involved in salivary gland development [GO:0060692] (BP) Definition: The process in which a relatively unspecialized cell acquires specialized features of a mesenchymal cell of the salivary gland. A mesenchymal cell is a loosely associated cell that is part of the connective tissue in an organism. Mesenchymal cells give rise to more mature connective tissue cell types. Sources: GOC:dph Relationships: is a type of mesenchymal cell differentiation [GO:0048762]; is a type of cell differentiation involved in salivary gland development [GO:0060689]